spindle midzone assembly [GO:0051255] (biological process) Also known as: spindle midzone biogenesis, spindle midzone biosynthesis, spindle midzone formation Definition: The cell cycle process in which aggregation, arrangement and bonding together of a set of components to form the spindle midzone. The spindle midzone is the area in the center of the spindle where the spindle microtubules from opposite poles overlap. References: PMID:15296749 Sources: GOC:ai Subtypes: GO:0051256, meiotic spindle midzone assembly [GO:0051257] Relationships: is a type of microtubule-based process [GO:0007017]; is a type of GO:0022402; is a type of cellular component assembly [GO:0022607]; is part of GO:0051225